{
  "gene_symbol": "VENTX",
  "term_label": "nucleus",
  "term_id": "GO:0005634",
  "gene_name": "Homeobox protein VENTX",
  "gene": "UniProtKB:O95231"
}